{
  "term_label": "cytoplasm",
  "gene_name": "Death-associated protein kinase 3",
  "gene": "UniProtKB:O43293",
  "term_id": "GO:0005737",
  "gene_symbol": "DAPK3"
}